{
  "gene_symbol": "OR2T27",
  "gene": "UniProtKB:Q8NH04",
  "term_id": "GO:0050911",
  "term_label": "detection of chemical stimulus involved in sensory perception of smell",
  "gene_name": "Olfactory receptor 2T27"
}